{
  "gene_symbol": "ZBTB6",
  "term_label": "negative regulation of transcription by RNA polymerase II",
  "gene": "UniProtKB:Q15916",
  "term_id": "GO:0000122",
  "gene_name": "Zinc finger and BTB domain-containing protein 6"
}